{
  "term_id": "GO:0003994",
  "gene_symbol": "ACO2",
  "term_label": "aconitate hydratase activity",
  "gene_name": "Aconitate hydratase, mitochondrial",
  "gene": "UniProtKB:Q99798"
}